akinete formation [GO:0034302] (biological process) Definition: The process in which an akinete, a thick-walled (encysted) dormant cell derived from the enlargement of a vegetative cell, is formed. Akinetes typically have granular cytoplasm, are more resistant to environmental extremes than vegetative cells, and are characteristic of several groups of Cyanobacteria. Relationships: is a type of asexual sporulation resulting in formation of a cellular spore [GO:0043936] References: PMID:11948167 Sources: GOC:ds, GOC:mah, https://doi.org/10.1016/S1369-703X(02)00136-5